{
  "gene_symbol": "KYAT1",
  "gene_name": "Kynurenine--oxoglutarate transaminase 1",
  "gene": "UniProtKB:Q16773",
  "term_label": "cytoplasm",
  "term_id": "GO:0005737"
}